ProVWX complex [GO:1990222] (cellular component) Relationships: is a type of ATP-binding cassette (ABC) transporter complex [GO:0043190] Definition: The ProVWX complex belongs to the family of ATP-binding cassette (ABC) transporter proteins complexes. It consists of a cytoplasmic ATPase subunit ProV, a transmembrane subunit ProW and a periplasmic binding protein ProX. It is capable of translocating a wide variety of solute (e.g. glycine betaine) across the plasma membrane and is activated under osmotic stress conditions. Also known as: ATP-binding cassette (ABC) transporter complex ProVWX References: PMID:23249124 Sources: GOC:bhm